{
  "term_label": "nuclear import signal receptor activity",
  "term_id": "GO:0061608",
  "gene_name": "Importin-4",
  "gene_symbol": "IPO4",
  "gene": "UniProtKB:Q8TEX9"
}